regulation of endothelial cell apoptotic process [GO:2000351] (biological process) Definition: Any process that modulates the frequency, rate or extent of endothelial cell apoptotic process. Also known as: regulation of apoptosis of endothelial cells, regulation of endothelial cell programmed cell death by apoptosis, regulation of killing of endothelial cells, regulation of programmed cell death of endothelial cells by apoptosis, regulation of programmed cell death, endothelial cells, regulation of endothelial cell apoptosis Subtypes: negative regulation of endothelial cell apoptotic process [GO:2000352], positive regulation of endothelial cell apoptotic process [GO:2000353] Relationships: is a type of regulation of apoptotic process [GO:0042981]; regulates endothelial cell apoptotic process [GO:0072577] Sources: GOC:mah, GOC:mtg_apoptosis